phototropism [GO:0009638] (biological process) References: PMID:16870491 Sources: GOC:jl, GOC:mtg_far_red Relationships: is a type of tropism [GO:0009606]; is a type of response to blue light [GO:0009637] Definition: The movement of an organism, or part of an organism, in response to a light stimulus, usually toward or away from it.